{
  "gene_name": "POU domain, class 3, transcription factor 4",
  "gene_symbol": "POU3F4",
  "gene": "UniProtKB:P49335",
  "term_label": "Unknown cellular component",
  "term_id": "UNKNOWN:0003"
}